AIP1-IRE1 complex [GO:1990597] (cellular component) Relationships: is a type of protein-containing complex [GO:0032991] References: PMID:18281285 Sources: GOC:PARL, GOC:bf Also known as: IRE1-DAB2IP complex, IRE1alpha-AIP1 complex, AIP1-ERN1 complex Definition: A protein complex consisting of IRE1 (inositol-requiring enzyme-1) bound to AIP1 (ASK1-interacting protein 1/DAB2-interacting protein).